{
  "gene": "UniProtKB:Q14165",
  "gene_name": "Malectin",
  "term_id": "GO:0016020",
  "gene_symbol": "MLEC",
  "term_label": "membrane"
}